myosin head/neck binding [GO:0032028] (molecular function) Definition: Binding to the head/neck region of a myosin heavy chain. Relationships: is_a myosin heavy chain binding [GO:0032036] Subtypes: myosin I head/neck binding [GO:0032031], GO:0032034, myosin VI head/neck binding [GO:0070855] Sources: GOC:mah